{
  "gene_symbol": "CCL13",
  "gene": "UniProtKB:Q99616",
  "gene_name": "C-C motif chemokine 13",
  "term_id": "GO:0061844",
  "term_label": "antimicrobial humoral immune response mediated by antimicrobial peptide"
}